{
  "term_id": "GO:0005125",
  "gene_name": "Bone morphogenetic protein 8B",
  "term_label": "cytokine activity",
  "gene": "UniProtKB:P34820",
  "gene_symbol": "BMP8B"
}